{
  "gene_name": "Uncharacterized protein C20orf202",
  "term_id": "UNKNOWN:0002",
  "gene_symbol": "C20orf202",
  "gene": "UniProtKB:A1L168",
  "term_label": "Unknown biological process"
}